{
  "gene_name": "High mobility group protein HMG-I_HMG-Y",
  "gene_symbol": "HMGA1",
  "term_label": "transcription coregulator activity",
  "gene": "UniProtKB:P17096",
  "term_id": "GO:0003712"
}